{
  "gene_name": "Calcium-transporting ATPase type 2C member 2",
  "gene": "UniProtKB:O75185",
  "term_label": "manganese ion transport",
  "term_id": "GO:0006828",
  "gene_symbol": "ATP2C2"
}